{
  "term_label": "Cul3-RING ubiquitin ligase complex",
  "gene_symbol": "KLHL42",
  "gene_name": "Kelch-like protein 42",
  "term_id": "GO:0031463",
  "gene": "UniProtKB:Q9P2K6"
}